pentadecane biosynthetic process [GO:1900634] (BP) Also known as: pentadecane anabolism, pentadecane biosynthesis, pentadecane formation, pentadecane synthesis Sources: GOC:TermGenie, GOC:mengo_curators Regulation: RO_0002211 by GO:1900887; negatively regulated by negative regulation of pentadecane biosynthetic process [GO:1900888]; RO_0002213 by positive regulation of pentadecane biosynthetic process [GO:1900889] Definition: The chemical reactions and pathways resulting in the formation of pentadecane. Relationships: is a type of GO:0043447; is a type of GO:1900633